transverse filament [GO:0000802] (cellular component) Definition: A structural unit of the synaptonemal complex that spans the regions between the lateral elements and connects them. Relationships: is a type of GO:0110165; is part of synaptonemal complex [GO:0000795] Sources: GOC:elh